ABC-type D-methionine transporter activity [GO:0033232] (molecular function) Definition: Enables the transfer of a solute or solutes from one side of a membrane to the other according to the reaction: ATP + H2O + D-methionine(out/in) = ADP + phosphate + D-methionine(in/out). References: PMID:12169620, PMID:12819857, PMID:18621668 Sources: GOC:mlg, RHEA:29767 Also known as: ATP-dependent D-methionine transporter activity, ATP-dependent methionine transmembrane transporter activity, ATPase-coupled D-methionine transporter activity, ATPase-coupled methionine transmembrane transporter activity, D-methionine exporter, D-methionine importer, D-methionine transmembrane transporter activity, D-methionine transporter activity, D-methionine-exporting ATPase activity, D-methionine-importing ATPase activity, D-methionine-transporting ATPase activity, methionine transmembrane-transporting ATPase activity Relationships: is a type of ABC-type amino acid transporter activity [GO:0015424]; is a type of ATPase-coupled carboxylic acid transmembrane transporter activity [GO:0033284]; is a type of D-amino acid transmembrane transporter activity [GO:0042943]; is a type of methionine transmembrane transporter activity [GO:0043865]; is part of D-methionine transmembrane transport [GO:0048473]